{
  "gene_name": "Zinc finger protein 24",
  "term_id": "GO:0000978",
  "term_label": "RNA polymerase II cis-regulatory region sequence-specific DNA binding",
  "gene": "UniProtKB:P17028",
  "gene_symbol": "ZNF24"
}